{
  "term_id": "GO:0072659",
  "gene": "UniProtKB:Q05513",
  "gene_name": "Protein kinase C zeta type",
  "gene_symbol": "PRKCZ",
  "term_label": "protein localization to plasma membrane"
}